{
  "term_id": "UNKNOWN:0002",
  "gene": "UniProtKB:Q6ZMB5",
  "term_label": "Unknown biological process",
  "gene_name": "Transmembrane protein 184A",
  "gene_symbol": "TMEM184A"
}